{
  "gene_symbol": "SEMA4B",
  "gene": "UniProtKB:Q9NPR2",
  "term_id": "GO:0050919",
  "term_label": "negative chemotaxis",
  "gene_name": "Semaphorin-4B"
}